{
  "term_label": "Unknown biological process",
  "gene_symbol": "ERVK11-1",
  "gene_name": "Putative endogenous retrovirus group K member 11-1 Env polyprotein",
  "gene": "UniProtKB:P61568",
  "term_id": "UNKNOWN:0002"
}